protein polyglutamylation [GO:0018095] (biological process) Sources: RESID:AA0202 Relationships: is a type of peptidyl-glutamic acid modification [GO:0018200] Definition: The addition of one or more alpha-linked glutamyl units to the gamma carboxyl group of peptidyl-glutamic acid.